{
  "gene": "UniProtKB:Q6ZN32",
  "term_label": "regulation of transcription by RNA polymerase II",
  "gene_symbol": "ETV3L",
  "gene_name": "ETS translocation variant 3-like protein",
  "term_id": "GO:0006357"
}